{
  "gene": "UniProtKB:P51452",
  "term_label": "cytosol",
  "gene_name": "Dual specificity protein phosphatase 3",
  "term_id": "GO:0005829",
  "gene_symbol": "DUSP3"
}